{
  "gene_symbol": "LTB4R2",
  "gene_name": "Leukotriene B4 receptor 2",
  "term_label": "neuropeptide signaling pathway",
  "gene": "UniProtKB:Q9NPC1",
  "term_id": "GO:0007218"
}